{
  "gene_name": "RNA-binding protein with multiple splicing",
  "gene": "UniProtKB:Q93062",
  "term_label": "mRNA binding",
  "term_id": "GO:0003729",
  "gene_symbol": "RBPMS"
}